{
  "gene_symbol": "ZSCAN2",
  "gene_name": "Zinc finger and SCAN domain-containing protein 2",
  "gene": "UniProtKB:Q7Z7L9",
  "term_id": "GO:0000977",
  "term_label": "RNA polymerase II transcription regulatory region sequence-specific DNA binding"
}